{
  "gene_name": "Trafficking kinesin-binding protein 2",
  "gene": "UniProtKB:O60296",
  "term_id": "GO:0047496",
  "gene_symbol": "TRAK2",
  "term_label": "vesicle transport along microtubule"
}